{
  "gene": "UniProtKB:Q9GZP8",
  "term_id": "UNKNOWN:0003",
  "gene_symbol": "IMUP",
  "term_label": "Unknown cellular component",
  "gene_name": "Immortalization up-regulated protein"
}